phosphate ion export across plasma membrane [GO:0180029] (biological process) References: PMID:37949217 Definition: The directed movement of phosphate ions (Pi) from inside of a cell, across the plasma membrane and into the extracellular region. Relationships: is a type of phosphate ion transmembrane transport [GO:0035435]; is a type of export across plasma membrane [GO:0140115]